{
  "gene_name": "Protein bicaudal D homolog 2",
  "gene": "UniProtKB:Q8TD16",
  "gene_symbol": "BICD2",
  "term_id": "GO:0070840",
  "term_label": "dynein complex binding"
}